regulation of intermediate mesodermal cell fate determination [GO:0048395] (biological process) Subtypes: negative regulation of intermediate mesodermal cell fate determination [GO:0048396], positive regulation of intermediate mesodermal cell fate determination [GO:0048397] Relationships: is a type of GO:0048334; regulates intermediate mesodermal cell fate determination [GO:0048394] Sources: GOC:dgh Definition: Any process that modulates the frequency, rate or extent of intermediate mesoderm cell fate determination.